{
  "term_label": "histone deacetylase activity",
  "gene": "UniProtKB:Q9BY41",
  "term_id": "GO:0004407",
  "gene_symbol": "HDAC8",
  "gene_name": "Histone deacetylase 8"
}